{
  "gene": "UniProtKB:Q5SQI0",
  "term_label": "Unknown cellular component",
  "gene_name": "Alpha-tubulin N-acetyltransferase 1",
  "gene_symbol": "ATAT1",
  "term_id": "UNKNOWN:0003"
}